{
  "gene": "UniProtKB:P00846",
  "gene_symbol": "MT-ATP6",
  "term_label": "proton motive force-driven ATP synthesis",
  "gene_name": "ATP synthase subunit a",
  "term_id": "GO:0015986"
}